{
  "gene_name": "Transcription factor ATOH8",
  "term_label": "positive regulation of transcription by RNA polymerase II",
  "gene": "UniProtKB:Q96SQ7",
  "term_id": "GO:0045944",
  "gene_symbol": "ATOH8"
}